{
  "gene_name": "Bromodomain-containing protein 3",
  "term_id": "GO:0000785",
  "term_label": "chromatin",
  "gene_symbol": "BRD3",
  "gene": "UniProtKB:Q15059"
}